{
  "gene": "UniProtKB:P15088",
  "gene_symbol": "CPA3",
  "term_id": "GO:0006508",
  "term_label": "proteolysis",
  "gene_name": "Mast cell carboxypeptidase A"
}